{
  "gene_name": "Thyroid receptor-interacting protein 6",
  "term_id": "GO:0007165",
  "gene_symbol": "TRIP6",
  "gene": "UniProtKB:Q15654",
  "term_label": "signal transduction"
}